{
  "term_label": "alkaline phosphatase activity",
  "gene_symbol": "ALPL",
  "gene": "UniProtKB:P05186",
  "term_id": "GO:0004035",
  "gene_name": "Alkaline phosphatase, tissue-nonspecific isozyme"
}